phorbol-diester hydrolase activity [GO:0050181] (molecular function) Also known as: 12,13-diacylphorbate 12-acylhydrolase activity, PDEH, diacylphorbate 12-hydrolase activity, phorbol-12,13-diester 12-ester hydrolase activity Relationships: is a type of carboxylic ester hydrolase activity [GO:0052689] Definition: Catalysis of the reaction: H2O + phorbol 12,13-dibutanoate = butanoate + H+ + phorbol 13-butanoate. Sources: EC:3.1.1.51, RHEA:21316